phosphate ion transmembrane transport [GO:0035435] (biological process) Definition: The process in which a phosphate is transported across a membrane. Sources: GOC:vw Also known as: phosphate ion membrane transport Note: Note that this term is not intended for use in annotating lateral movement within membranes. Relationships: is a type of phosphate ion transport [GO:0006817]; is a type of GO:0055085 Subtypes: GO:0180029, transmembrane phosphate ion transport from cytosol to vacuole [GO:1905011], mitochondrial phosphate ion transmembrane transport [GO:1990547] Regulation: regulated by regulation of phosphate transmembrane transport [GO:2000185]; negatively regulated by negative regulation of phosphate transmembrane transport [GO:2000186]; positively regulated by GO:2000187